cellular response to gold(3+) [GO:1904312] (biological process) Relationships: is_a cellular response to metal ion [GO:0071248]; is a type of GO:1904311 Definition: Any process that results in a change in state or activity of a cell (in terms of movement, secretion, enzyme production, gene expression, etc.) as a result of a gold(3+) stimulus. References: PMID:16206274 Sources: GOC:TermGenie, GO_REF:0000071